{
  "gene_symbol": "RNF183",
  "gene": "UniProtKB:Q96D59",
  "gene_name": "E3 ubiquitin-protein ligase RNF183",
  "term_label": "ubiquitin protein ligase activity",
  "term_id": "GO:0061630"
}